receptor tyrosine kinase-like orphan receptor binding [GO:0005115] (molecular function) Definition: Binding to a receptor tyrosine kinase-like orphan receptor (Ror). Sources: GOC:ceb, GOC:vw Also known as: Ror binding, receptor tyrosine kinase-like orphan receptor ligand, Ror ligand Relationships: is a type of GO:0005102